{
  "gene": "UniProtKB:Q8NGX1",
  "term_label": "olfactory receptor activity",
  "gene_symbol": "OR2T34",
  "gene_name": "Olfactory receptor 2T34",
  "term_id": "GO:0004984"
}